{
  "gene_symbol": "CACNG7",
  "gene_name": "Voltage-dependent calcium channel gamma-7 subunit",
  "gene": "UniProtKB:P62955",
  "term_id": "GO:0019226",
  "term_label": "transmission of nerve impulse"
}